{
  "gene_symbol": "PLXNB2",
  "gene_name": "Plexin-B2",
  "term_label": "positive regulation of axonogenesis",
  "term_id": "GO:0050772",
  "gene": "UniProtKB:O15031"
}